CCR chemokine receptor binding [GO:0048020] (molecular function) Subtypes: CCR1 chemokine receptor binding [GO:0031726], CCR2 chemokine receptor binding [GO:0031727], CCR3 chemokine receptor binding [GO:0031728], GO:0031729, GO:0031730, CCR6 chemokine receptor binding [GO:0031731], CCR7 chemokine receptor binding [GO:0031732], CCR8 chemokine receptor binding [GO:0031733], GO:0031734, GO:0031735, CCR11 chemokine receptor binding [GO:0031736] Definition: Binding to a CCR chemokine receptor. Sources: GOC:ai Relationships: is a type of chemokine receptor binding [GO:0042379] Also known as: beta chemokine receptor binding, CCR chemokine receptor ligand, beta chemokine receptor ligand